{
  "gene_symbol": "CST9",
  "gene": "UniProtKB:Q5W186",
  "gene_name": "Cystatin-9",
  "term_id": "GO:0019730",
  "term_label": "antimicrobial humoral response"
}